{
  "gene_name": "Phospholipase A2 group V",
  "gene": "UniProtKB:P39877",
  "term_label": "calcium-dependent phospholipase A2 activity",
  "term_id": "GO:0047498",
  "gene_symbol": "PLA2G5"
}